{
  "term_label": "double-strand break repair via homologous recombination",
  "gene_name": "SOSS complex subunit B2",
  "gene_symbol": "NABP1",
  "term_id": "GO:0000724",
  "gene": "UniProtKB:Q96AH0"
}